7SK snRNA binding [GO:0097322] (molecular function) Definition: Binding to a 7SK small nuclear RNA (7SK snRNA). Also known as: 7SK small nuclear RNA binding References: PMID:21853533 Sources: GOC:nhn Relationships: is a type of GO:0017069